{
  "term_label": "protein O-linked glycosylation",
  "gene_name": "Polypeptide N-acetylgalactosaminyltransferase 10",
  "gene": "UniProtKB:Q86SR1",
  "gene_symbol": "GALNT10",
  "term_id": "GO:0006493"
}